{
  "gene": "UniProtKB:Q16650",
  "gene_name": "T-box brain protein 1",
  "term_id": "GO:0001708",
  "gene_symbol": "TBR1",
  "term_label": "cell fate specification"
}